{
  "term_label": "serotonin-gated monoatomic cation channel activity",
  "gene": "UniProtKB:Q8WXA8",
  "gene_name": "5-hydroxytryptamine receptor 3C",
  "term_id": "GO:0022850",
  "gene_symbol": "HTR3C"
}